positive regulation of cytochrome-c oxidase activity [GO:1904960] (biological process) Definition: Any process that activates or increases the frequency, rate or extent of cytochrome-c oxidase activity. Relationships: is a type of GO:0032414; is a type of regulation of cytochrome-c oxidase activity [GO:1904959]; RO_0002213 cytochrome-c oxidase activity [GO:0004129] Also known as: positive regulation of NADH cytochrome c oxidase, positive regulation of cytochrome c oxidase activity, up regulation of NADH cytochrome c oxidase, up regulation of cytochrome c oxidase activity, up regulation of cytochrome-c oxidase activity, up-regulation of NADH cytochrome c oxidase, up-regulation of cytochrome c oxidase activity, up-regulation of cytochrome-c oxidase activity, upregulation of NADH cytochrome c oxidase, upregulation of cytochrome c oxidase activity, upregulation of cytochrome-c oxidase activity, activation of NADH cytochrome c oxidase, activation of aa3-type cytochrome c oxidase, activation of ba3-type cytochrome c oxidase, activation of caa3-type cytochrome c oxidase, activation of cbb3-type cytochrome c oxidase, activation of cytochrome a3 activity, activation of cytochrome aa3 activity, activation of cytochrome c oxidase activity, activation of cytochrome-c oxidase activity, activation of ferrocytochrome c oxidase, activation of ferrocytochrome-c:oxygen oxidoreductase, activation of indophenol oxidase, activation of indophenolase, positive regulation of aa3-type cytochrome c oxidase, positive regulation of ba3-type cytochrome c oxidase, positive regulation of caa3-type cytochrome c oxidase, positive regulation of cbb3-type cytochrome c oxidase, positive regulation of cytochrome a3 activity, positive regulation of cytochrome aa3 activity, positive regulation of ferrocytochrome c oxidase, positive regulation of ferrocytochrome-c:oxygen oxidoreductase, positive regulation of indophenol oxidase, positive regulation of indophenolase, up regulation of aa3-type cytochrome c oxidase, up regulation of ba3-type cytochrome c oxidase, up regulation of caa3-type cytochrome c oxidase, up regulation of cbb3-type cytochrome c oxidase, up regulation of cytochrome a3 activity, up regulation of cytochrome aa3 activity, up regulation of ferrocytochrome c oxidase, up regulation of ferrocytochrome-c:oxygen oxidoreductase, up regulation of indophenol oxidase, up regulation of indophenolase, up-regulation of aa3-type cytochrome c oxidase, up-regulation of ba3-type cytochrome c oxidase, up-regulation of caa3-type cytochrome c oxidase, up-regulation of cbb3-type cytochrome c oxidase, up-regulation of cytochrome a3 activity, up-regulation of cytochrome aa3 activity, up-regulation of ferrocytochrome c oxidase, up-regulation of ferrocytochrome-c:oxygen oxidoreductase, up-regulation of indophenol oxidase, up-regulation of indophenolase, upregulation of aa3-type cytochrome c oxidase, upregulation of ba3-type cytochrome c oxidase, upregulation of caa3-type cytochrome c oxidase, upregulation of cbb3-type cytochrome c oxidase, upregulation of cytochrome a3 activity, upregulation of cytochrome aa3 activity, upregulation of ferrocytochrome c oxidase, upregulation of ferrocytochrome-c:oxygen oxidoreductase, upregulation of indophenol oxidase, upregulation of indophenolase, activation of complex IV (mitochondrial electron transport) activity, activation of cytochrome oxidase activity, activation of warburg's respiratory enzyme activity, positive regulation of complex IV (mitochondrial electron transport) activity, positive regulation of cytochrome oxidase activity, positive regulation of warburg's respiratory enzyme activity, up regulation of complex IV (mitochondrial electron transport) activity, up regulation of cytochrome oxidase activity, up regulation of warburg's respiratory enzyme activity, up-regulation of complex IV (mitochondrial electron transport) activity, up-regulation of cytochrome oxidase activity, up-regulation of warburg's respiratory enzyme activity, upregulation of complex IV (mitochondrial electron transport) activity, upregulation of cytochrome oxidase activity, upregulation of warburg's respiratory enzyme activity References: PMID:26734017 Sources: GOC:TermGenie, GO_REF:0000059